{
  "term_id": "UNKNOWN:0001",
  "gene_symbol": "C1GALT1C1",
  "term_label": "Unknown molecular function",
  "gene": "UniProtKB:Q96EU7",
  "gene_name": "C1GALT1-specific chaperone 1"
}